{
  "term_id": "GO:0004890",
  "gene": "UniProtKB:Q16445",
  "term_label": "GABA-A receptor activity",
  "gene_name": "Gamma-aminobutyric acid receptor subunit alpha-6",
  "gene_symbol": "GABRA6"
}